{
  "term_id": "GO:0004674",
  "term_label": "protein serine/threonine kinase activity",
  "gene": "UniProtKB:Q9UQ88",
  "gene_symbol": "CDK11A",
  "gene_name": "Cyclin-dependent kinase 11A"
}